{
  "gene_symbol": "SPATA31A1",
  "term_id": "UNKNOWN:0002",
  "gene": "UniProtKB:Q5TZJ5",
  "term_label": "Unknown biological process",
  "gene_name": "Spermatogenesis-associated protein 31A1"
}